{
  "gene_symbol": "SHANK1",
  "gene": "UniProtKB:Q9Y566",
  "term_label": "synaptic receptor adaptor activity",
  "gene_name": "SH3 and multiple ankyrin repeat domains protein 1",
  "term_id": "GO:0030160"
}